{
  "gene_symbol": "IGLJ5",
  "term_id": "UNKNOWN:0003",
  "term_label": "Unknown cellular component",
  "gene": "UniProtKB:A0A0A0MT86",
  "gene_name": "Immunoglobulin lambda joining 5 (non-functional) (Fragment)"
}